thiol S-methyltransferase activity [GO:0018708] (molecular function) Also known as: S-adenosyl-L-methionine:thiol S-methyltransferase activity, TMT, thiol methyltransferase activity Relationships: is a type of S-methyltransferase activity [GO:0008172]; is a type of S-adenosylmethionine-dependent methyltransferase activity [GO:0008757] Sources: EC:2.1.1.9 Definition: Catalysis of the reaction: S-adenosyl-L-methionine + a thiol = S-adenosyl-L-homocysteine + a thioether.